mitral valve formation [GO:0003192] (biological process) Relationships: is a type of atrioventricular valve formation [GO:0003190]; is part of GO:0003183 Definition: The developmental process pertaining to the initial formation of the mitral valve from unspecified parts. This process begins with the specific processes that contribute to the appearance of the discrete structure and ends when the structural rudiment is recognizable. Sources: GOC:mtg_heart